{
  "term_id": "UNKNOWN:0002",
  "term_label": "Unknown biological process",
  "gene_name": "Mucin-1",
  "gene": "UniProtKB:P15941",
  "gene_symbol": "MUC1"
}